{
  "gene": "UniProtKB:A6NEE1",
  "gene_name": "Pleckstrin homology domain-containing family D member 1",
  "gene_symbol": "PLEKHD1",
  "term_label": "Unknown molecular function",
  "term_id": "UNKNOWN:0001"
}